D-allose biosynthetic process [GO:0019315] (biological process) Definition: The chemical reactions and pathways resulting in the formation of D-allose, the D-enantiomer of allo-hexose, an aldohexose similar to glucose. Sources: GOC:ai, GOC:jsg, GOC:mah Relationships: is a type of GO:0019319 Also known as: D-allose anabolism, D-allose biosynthesis, D-allose formation, D-allose synthesis